phylloquinone biosynthetic process [GO:0042372] (biological process) Relationships: is a type of vitamin K biosynthetic process [GO:0042371] Definition: The chemical reactions and pathways resulting in the formation of phylloquinone, vitamin K1, a quinone-derived compound synthesized by green plants. References: PMID:23821151, PMID:27337968 Sources: GOC:jl, https://doi.org/10.1016/B978-0-12-385853-5.00001-5 Also known as: phylloquinone anabolism, phylloquinone biosynthesis, phylloquinone formation, phylloquinone synthesis, phytomenadione biosynthesis, phytomenadione biosynthetic process, phytonadione biosynthesis, phytonadione biosynthetic process, phytylmenaquinone biosynthesis, phytylmenaquinone biosynthetic process, vitamin K1 biosynthesis, vitamin K1 biosynthetic process